{
  "gene_name": "Putative sodium-coupled neutral amino acid transporter 8",
  "gene": "UniProtKB:A6NNN8",
  "gene_symbol": "SLC38A8",
  "term_label": "membrane",
  "term_id": "GO:0016020"
}